{
  "gene_symbol": "CLSTN2",
  "gene_name": "Calsyntenin-2",
  "term_id": "GO:0098632",
  "term_label": "cell-cell adhesion mediator activity",
  "gene": "UniProtKB:Q9H4D0"
}